{
  "gene": "UniProtKB:Q96PP8",
  "gene_name": "Guanylate-binding protein 5",
  "term_label": "cellular response to type II interferon",
  "term_id": "GO:0071346",
  "gene_symbol": "GBP5"
}